{
  "term_id": "GO:0005635",
  "gene_name": "Glutathione S-transferase 3, mitochondrial",
  "term_label": "nuclear envelope",
  "gene_symbol": "MGST3",
  "gene": "UniProtKB:O14880"
}